{
  "gene_symbol": "LSM10",
  "gene_name": "U7 snRNA-associated Sm-like protein LSm10",
  "term_label": "nuclear body",
  "term_id": "GO:0016604",
  "gene": "UniProtKB:Q969L4"
}